{
  "gene_name": "SLIT-ROBO Rho GTPase-activating protein 2C",
  "gene": "UniProtKB:P0DJJ0",
  "term_id": "GO:0051963",
  "gene_symbol": "SRGAP2C",
  "term_label": "regulation of synapse assembly"
}